regulation of cell communication by chemical coupling [GO:0010645] (biological process) Relationships: is a type of regulation of cell communication [GO:0010646]; regulates cell communication by chemical coupling [GO:0010643] Definition: Any process that modulates the frequency, rate or extent of cell communication via chemical coupling. Cell communication by chemical coupling is the process that mediates signaling interactions between one cell and another cell by the transfer of small, water-soluble molecules or metabolites between their adjacent cytoplasms via intercellular protein channels. Subtypes: positive regulation of cell communication by chemical coupling [GO:0010652], negative regulation of cell communication by chemical coupling [GO:0010653] Sources: GOC:dph, GOC:kmv, GOC:tb